regulation of transcription by RNA polymerase I [GO:0006356] (biological process) Definition: Any process that modulates the frequency, rate or extent of transcription mediated by RNA polymerase I. Sources: GOC:go_curators Also known as: regulation of transcription from Pol I promoter, regulation of transcription from RNA polymerase I promoter Relationships: is a type of regulation of DNA-templated transcription [GO:0006355]; regulates GO:0006360 Subtypes: negative regulation of transcription by RNA polymerase I [GO:0016479], positive regulation of transcription by RNA polymerase I [GO:0045943], regulation of transcription of nucleolar large rRNA by RNA polymerase I [GO:1901836], regulation of transcription initiation by RNA polymerase I [GO:1903357], regulation of termination of RNA polymerase I transcription [GO:2000730]